{
  "term_label": "protein K6-linked ubiquitination",
  "gene_symbol": "BARD1",
  "gene": "UniProtKB:Q99728",
  "term_id": "GO:0085020",
  "gene_name": "BRCA1-associated RING domain protein 1"
}